imidazolone hydrolase activity [GO:0043804] (molecular function) Definition: Catalysis of the reaction: imidazol-4-one + H2O = N-formimidoylglycine. References: PMID:27286964 Sources: RHEA:24935 Note: Note that this reaction can occur spontaneously (see RHEA:24937). Relationships: is a type of hydrolase activity, acting on carbon-nitrogen (but not peptide) bonds, in cyclic amides [GO:0016812]